imidazoleacetate-phosphoribosyldiphosphate ligase activity [GO:0047483] (molecular function) Also known as: 5-phosphoribosylimidazoleacetate synthetase activity, imidazoleacetate:5-phosphoribosyl-diphosphate ligase (ADP- and diphosphate-forming) Sources: EC:6.3.4.8, RHEA:16485 Definition: Catalysis of the reaction: 5-phospho-alpha-D-ribose 1-diphosphate + ATP + H2O + imidazol-4-ylacetate = 1-(5-phosphoribosyl)imidazol-4-ylacetate + ADP + diphosphate + 2 H+ + phosphate. Relationships: is a type of ligase activity, forming carbon-nitrogen bonds [GO:0016879]